{
  "term_id": "GO:1990756",
  "gene_name": "F-box_SPRY domain-containing protein 1",
  "term_label": "ubiquitin-like ligase-substrate adaptor activity",
  "gene": "UniProtKB:P0C2W1",
  "gene_symbol": "FBXO45"
}